{
  "term_label": "cytosol",
  "gene_name": "Serine_threonine-protein phosphatase 5",
  "gene": "UniProtKB:P53041",
  "term_id": "GO:0005829",
  "gene_symbol": "PPP5C"
}